{
  "term_id": "GO:0036064",
  "gene": "UniProtKB:Q8WYA0",
  "gene_symbol": "IFT81",
  "term_label": "ciliary basal body",
  "gene_name": "Intraflagellar transport protein 81 homolog"
}